{
  "gene_symbol": "MORN3",
  "gene": "UniProtKB:Q6PF18",
  "term_id": "UNKNOWN:0002",
  "term_label": "Unknown biological process",
  "gene_name": "MORN repeat-containing protein 3"
}